{
  "term_label": "nucleus",
  "term_id": "GO:0005634",
  "gene_symbol": "FOXP4",
  "gene_name": "Forkhead box protein P4",
  "gene": "UniProtKB:Q8IVH2"
}